{
  "gene_symbol": "C2CD5",
  "gene_name": "C2 domain-containing protein 5",
  "term_label": "calcium ion binding",
  "gene": "UniProtKB:Q86YS7",
  "term_id": "GO:0005509"
}